{
  "term_id": "UNKNOWN:0002",
  "gene_symbol": "C16orf96",
  "term_label": "Unknown biological process",
  "gene": "UniProtKB:A6NNT2",
  "gene_name": "Uncharacterized protein C16orf96"
}